mitotic G1/S transition checkpoint signaling [GO:0044819] (biological process) Sources: GOC:mtg_cell_cycle Relationships: is a type of GO:0007093; is a type of negative regulation of G1/S transition of mitotic cell cycle [GO:2000134] Definition: A cell cycle checkpoint that detects and negatively regulates progression from G1 to S phase as part of a mitotic cell cycle. Also known as: mitotic G1/S transition checkpoint Subtypes: mitotic G1 DNA damage checkpoint signaling [GO:0031571]